{
  "gene": "UniProtKB:Q99603",
  "gene_name": "T cell receptor gamma variable 9",
  "term_id": "UNKNOWN:0002",
  "gene_symbol": "TRGV9",
  "term_label": "Unknown biological process"
}